{
  "term_label": "cell migration",
  "gene_name": "Guanine nucleotide exchange factor VAV2",
  "term_id": "GO:0016477",
  "gene": "UniProtKB:P52735",
  "gene_symbol": "VAV2"
}